{
  "gene": "UniProtKB:Q8NI38",
  "term_label": "Unknown molecular function",
  "gene_name": "NF-kappa-B inhibitor delta",
  "gene_symbol": "NFKBID",
  "term_id": "UNKNOWN:0001"
}